{
  "gene": "UniProtKB:Q9P0W8",
  "term_id": "GO:0036064",
  "gene_symbol": "SPATA7",
  "gene_name": "Spermatogenesis-associated protein 7",
  "term_label": "ciliary basal body"
}